cell adhesive protein binding involved in Purkinje myocyte-ventricular cardiac muscle cell communication [GO:0086084] (MF) Sources: GOC:BHF, GOC:mtg_cardiac_conduct_nov11 Definition: Binding to a protein or protein complex that results in the connection of a Purkinje myocyte with an ventricular cardiac muscle cell and contributes to the communication between the two cells. Relationships: is_a protein binding involved in heterotypic cell-cell adhesion [GO:0086080]; is part of GO:0086074